amylin receptor 2 signaling pathway [GO:0150060] (biological process) Also known as: AMY2 signaling pathway References: PMID:22500019 Sources: GOC:aruk, GOC:bc Relationships: is_a amylin receptor signaling pathway [GO:0097647] Definition: The series of molecular signals initiated by an extracellular amylin, or another ligand, combining with an amylin receptor 2 (AMY2), a G protein-coupled receptor complex, on the surface of the target cell. The AMY2 signaling pathway can also be initiated by adrenomedullin (AM/ADM).